platelet glycocalyx [GO:0120240] (cellular component) Relationships: is a type of glycocalyx [GO:0030112] References: PMID:24967889 Sources: GOC:krc Definition: The carbohydrate rich layer at the outermost periphery of a platelet.